{
  "gene_name": "Sperm surface protein Sp17",
  "gene_symbol": "SPA17",
  "term_label": "Unknown biological process",
  "gene": "UniProtKB:Q15506",
  "term_id": "UNKNOWN:0002"
}